negative regulation of cell growth involved in contact inhibition [GO:0060243] (biological process) Sources: GOC:dph Definition: The negative regulation of cell growth in response to increased cell density. Relationships: is a type of negative regulation of cell growth [GO:0030308]; is part of contact inhibition [GO:0060242]